{
  "gene_name": "Aldo-keto reductase family 1 member B15",
  "gene_symbol": "AKR1B15",
  "term_label": "mitochondrion",
  "gene": "UniProtKB:C9JRZ8",
  "term_id": "GO:0005739"
}